clathrin heavy chain binding [GO:0032050] (molecular function) Relationships: is a type of clathrin binding [GO:0030276] Definition: Binding to a clathrin heavy chain. Sources: GOC:mah